puparial adhesion [GO:0007594] (BP) Definition: The adhesion of the puparia of Diptera to their substrate; normally effected by a 'glue' secreted by the larval salivary gland and expectorated at the time of pupariation. Sources: GOC:ma Also known as: puparial glue Relationships: is a type of GO:0022609; is part of molting cycle, chitin-based cuticle [GO:0007591]